regulation of heart growth [GO:0060420] (biological process) Definition: Any process that modulates the rate or extent of heart growth. Heart growth is the increase in size or mass of the heart. Subtypes: regulation of cardiac muscle tissue growth [GO:0055021], positive regulation of heart growth [GO:0060421], GO:0061117 Relationships: is a type of regulation of organ growth [GO:0046620]; is_a regulation of multicellular organismal development [GO:2000026]; regulates GO:0060419 Sources: GOC:dph, GOC:tb